acetolactate decarboxylase activity [GO:0047605] (molecular function) Also known as: (S)-2-hydroxy-2-methyl-3-oxobutanoate carboxy-lyase [(R)-2-acetoin-forming], (S)-2-hydroxy-2-methyl-3-oxobutanoate carboxy-lyase activity, alpha-acetolactate decarboxylase activity Sources: EC:4.1.1.5, MetaCyc:ACETOLACTATE-DECARBOXYLASE-RXN Relationships: is a type of carboxy-lyase activity [GO:0016831] Definition: Catalysis of the reaction: (S)-2-hydroxy-2-methyl-3-oxobutanoate = (R)-2-acetoin + CO2.